{
  "gene_symbol": "LRP4",
  "gene_name": "Low-density lipoprotein receptor-related protein 4",
  "term_id": "GO:0048699",
  "term_label": "generation of neurons",
  "gene": "UniProtKB:O75096"
}